{
  "gene_symbol": "SIGLECL1",
  "gene_name": "SIGLEC family-like protein 1",
  "term_label": "Unknown biological process",
  "gene": "UniProtKB:Q8N7X8",
  "term_id": "UNKNOWN:0002"
}